{
  "gene": "UniProtKB:P01766",
  "gene_name": "Immunoglobulin heavy variable 3-13",
  "gene_symbol": "IGHV3-13",
  "term_id": "GO:0003823",
  "term_label": "antigen binding"
}